{
  "term_label": "glutamate metabolic process",
  "gene": "UniProtKB:Q7Z3D6",
  "term_id": "GO:0006536",
  "gene_symbol": "DGLUCY",
  "gene_name": "D-glutamate cyclase, mitochondrial"
}